{
  "term_id": "UNKNOWN:0002",
  "gene_name": "Gametocyte-specific factor 1-like",
  "gene": "UniProtKB:Q9H1H1",
  "term_label": "Unknown biological process",
  "gene_symbol": "GTSF1L"
}